dCTP metabolic process [GO:0046065] (biological process) Subtypes: GO:0006242, dCTP catabolic process [GO:0006253] Also known as: dCTP metabolism Sources: GOC:go_curators Definition: The chemical reactions and pathways involving dCTP, deoxycytidine triphosphate. Relationships: is a type of pyrimidine deoxyribonucleoside triphosphate metabolic process [GO:0009211]; is_a GO:0009219